alpha4-beta1 integrin-thrombospondin-2 complex [GO:0071070] (cellular component) References: PMID:11980922 Also known as: ITGA4-ITGB1-THBS2 complex Relationships: is a type of plasma membrane protein complex [GO:0098797] Definition: A protein complex that consists of an alpha4-beta1 integrin complex bound to thrombospondin-2.